regulation of timing of catagen [GO:0051794] (biological process) Definition: Any process that modulates the frequency, rate or extent of timing of catagen, the regression phase of the hair cycle. Relationships: is a type of regulation of hair follicle maturation [GO:0048819]; regulates catagen [GO:0042637] Sources: GOC:ai, GOC:pr Subtypes: positive regulation of timing of catagen [GO:0051795], negative regulation of timing of catagen [GO:0051796] Also known as: regulation of catagen